{
  "term_label": "Unknown molecular function",
  "gene_symbol": "ZNF2",
  "gene": "UniProtKB:Q9BSG1",
  "gene_name": "Zinc finger protein 2",
  "term_id": "UNKNOWN:0001"
}